{
  "gene": "UniProtKB:P0DV77",
  "term_label": "DNA-binding transcription factor activity, RNA polymerase II-specific",
  "term_id": "GO:0000981",
  "gene_name": "Tetrapeptide repeat homeobox protein 2",
  "gene_symbol": "TPRX2"
}